amphid sensory organ development [GO:0003386] (biological process) Definition: The progression of the amphid sensory organ over time, from its formation to the mature structure. Amphid sensory organs are the sensory organs of nematodes. Sources: GOC:ascb_2009, GOC:dph, GOC:tb Relationships: is_a sensory organ development [GO:0007423]